{
  "gene": "UniProtKB:Q02410",
  "gene_symbol": "APBA1",
  "term_label": "plasma membrane",
  "gene_name": "Amyloid-beta A4 precursor protein-binding family A member 1",
  "term_id": "GO:0005886"
}